regulation of ERAD pathway [GO:1904292] (biological process) Definition: Any process that modulates the frequency, rate or extent of ERAD pathway. Sources: GOC:PARL, GOC:TermGenie, GOC:bf, GO_REF:0000058 Also known as: regulation of endoplasmic reticulum-associated degradation, regulation of ER-associated degradation pathway, regulation of endoplasmic reticulum-associated protein degradation pathway Subtypes: negative regulation of ERAD pathway [GO:1904293], GO:1904294 Relationships: is a type of regulation of proteasomal protein catabolic process [GO:0061136]; is a type of regulation of response to endoplasmic reticulum stress [GO:1905897]; regulates ERAD pathway [GO:0036503]